GTP cyclohydrolase I activity [GO:0003934] (molecular function) Definition: Catalysis of the reaction: GTP + H2O = 7,8-dihydroneopterin 3'-triphosphate + formate + H+. Also known as: GTP 7,8-8,9-dihydrolase activity, GTP 8-formylhydrolase activity, dihydroneopterin triphosphate synthase activity, guanosine triphosphate 8-deformylase activity, guanosine triphosphate cyclohydrolase activity Sources: EC:3.5.4.16 Relationships: is a type of GTP cyclohydrolase activity [GO:0003933] Regulation: regulated by GTP cyclohydrolase I regulator activity [GO:0060308]